{
  "gene_name": "Polyadenylate-binding protein-interacting protein 2B",
  "term_label": "translation repressor activity",
  "gene": "UniProtKB:Q9ULR5",
  "term_id": "GO:0030371",
  "gene_symbol": "PAIP2B"
}